{
  "term_label": "lamellipodium",
  "gene_symbol": "MYLK",
  "term_id": "GO:0030027",
  "gene": "UniProtKB:Q15746",
  "gene_name": "Myosin light chain kinase, smooth muscle"
}